{
  "gene_name": "Glycine cleavage system H protein, mitochondrial",
  "gene": "UniProtKB:P23434",
  "gene_symbol": "GCSH",
  "term_label": "Unknown molecular function",
  "term_id": "UNKNOWN:0001"
}